{
  "gene": "UniProtKB:Q9NZM1",
  "term_label": "synaptic vesicle membrane",
  "term_id": "GO:0030672",
  "gene_name": "Myoferlin",
  "gene_symbol": "MYOF"
}